{
  "gene_name": "Kinase suppressor of Ras 2",
  "gene_symbol": "KSR2",
  "gene": "UniProtKB:Q6VAB6",
  "term_id": "GO:0007265",
  "term_label": "Ras protein signal transduction"
}